{
  "gene_name": "Protocadherin alpha-6",
  "term_id": "GO:0007155",
  "gene_symbol": "PCDHA6",
  "gene": "UniProtKB:Q9UN73",
  "term_label": "cell adhesion"
}